signaling receptor inhibitor activity [GO:0030547] (molecular function) Sources: GOC:ceb Definition: Binds to and modulates the activity of a signaling receptor. Subtypes: transmembrane receptor protein tyrosine kinase inhibitor activity [GO:0030293], GO:0030550, GO:0048019 Also known as: receptor inhibitor activity Relationships: is a type of GO:0030545; is a type of molecular function inhibitor activity [GO:0140678]; negatively regulates signaling receptor activity [GO:0038023]